{
  "gene": "UniProtKB:Q08257",
  "gene_symbol": "CRYZ",
  "gene_name": "Quinone oxidoreductase",
  "term_id": "UNKNOWN:0002",
  "term_label": "Unknown biological process"
}